{
  "gene_symbol": "RASSF9",
  "gene": "UniProtKB:O75901",
  "term_id": "UNKNOWN:0002",
  "term_label": "Unknown biological process",
  "gene_name": "Ras association domain-containing protein 9"
}